negative regulation of adenylate cyclase-inhibiting opioid receptor signaling pathway [GO:1900730] (biological process) Relationships: is a type of regulation of adenylate cyclase-inhibiting opioid receptor signaling pathway [GO:1900729]; is a type of GO:2000475; negatively regulates adenylate cyclase-inhibiting opioid receptor signaling pathway [GO:0031635] Definition: Any process that stops, prevents or reduces the frequency, rate or extent of adenylate cyclase-inhibiting opioid receptor signaling pathway. Also known as: down regulation of adenylate cyclase-inhibiting opioid receptor signaling pathway, down-regulation of adenylate cyclase-inhibiting opioid receptor signaling pathway, downregulation of adenylate cyclase-inhibiting opioid receptor signaling pathway, inhibition of adenylate cyclase-inhibiting opioid receptor signaling pathway, inhibition of opioid receptor-mediated adenylate cyclase inhibition, negative regulation of inhibition of adenylate cyclase activity by opioid receptor signaling pathway, negative regulation of inhibition of adenylate cyclase activity by opioid receptor signalling pathway References: PMID:17157995 Sources: GOC:TermGenie, GOC:sjw